bacterial-type flagellum motor [GO:0120100] (cellular component) References: PMID:10572114, PMID:12624192, PMID:24697492, PMID:25251856 Sources: DOI:10.1002/9780470015902.a0000744.pub4, GOC:cilia Relationships: is a type of cellular anatomical structure [GO:0110165]; is part of bacterial-type flagellum basal body [GO:0009425] Definition: A transmembrane complex embedded in the cytoplasmic membrane which is the motor force, or torque, generator of the bacterial-type flagellum. The motor consists of a membrane-anchored rotor complex surrounded by one or more stator complexes in the cytoplasmic membrane. The stator consists of a hetero-hexameric complex of 2 membrane proteins, A and B, with stoichiometry A4B2. Examples are the H+ driven MotA-MotB stator complex of Escherichia coli and Salmonella enterica, and the Na+ driven PomA-PomB stator complex of Vibrio and Shewanella species. The rotor complex consists of a membrane-anchored ring and the motor switch complex, which controls the direction of flagellar rotation.